{
  "gene": "UniProtKB:Q86YG4",
  "gene_symbol": "NT5DC4",
  "term_id": "UNKNOWN:0003",
  "term_label": "Unknown cellular component",
  "gene_name": "5'-nucleotidase domain-containing protein 4"
}